{
  "term_label": "Unknown molecular function",
  "gene_name": "Triple QxxK_R motif-containing protein",
  "term_id": "UNKNOWN:0001",
  "gene_symbol": "TRIQK",
  "gene": "UniProtKB:Q629K1"
}